{
  "term_label": "endosomal transport",
  "gene": "UniProtKB:Q9Y5X1",
  "gene_name": "Sorting nexin-9",
  "gene_symbol": "SNX9",
  "term_id": "GO:0016197"
}